alpha5-beta1 integrin-osteopontin complex [GO:0071128] (cellular component) Definition: A protein complex that consists of an alpha5-beta1 integrin complex bound to osteopontin. References: PMID:16005200 Also known as: ITGA5-ITGB1-SPP1 complex Relationships: is a type of plasma membrane protein complex [GO:0098797]